{
  "gene_symbol": "CLDN24",
  "gene_name": "Putative claudin-24",
  "term_id": "UNKNOWN:0002",
  "gene": "UniProtKB:A6NM45",
  "term_label": "Unknown biological process"
}